{
  "gene_name": "Tyrosine--tRNA ligase, cytoplasmic",
  "term_id": "GO:0004831",
  "term_label": "tyrosine-tRNA ligase activity",
  "gene_symbol": "YARS1",
  "gene": "UniProtKB:P54577"
}